{
  "gene": "UniProtKB:O00410",
  "gene_symbol": "IPO5",
  "term_label": "cytoplasm",
  "term_id": "GO:0005737",
  "gene_name": "Importin-5"
}